{
  "gene_name": "Structure-specific endonuclease subunit SLX1",
  "term_id": "GO:0000724",
  "term_label": "double-strand break repair via homologous recombination",
  "gene_symbol": "SLX1A",
  "gene": "UniProtKB:Q9BQ83"
}